positive regulation of methane biosynthetic process from dimethyl sulfide [GO:1900344] (biological process) Also known as: up regulation of methane biosynthetic process from dimethyl sulfide, up-regulation of methane biosynthetic process from dimethyl sulfide, upregulation of methane biosynthetic process from dimethyl sulfide, activation of methane biosynthetic process from dimethyl sulfide Relationships: is_a regulation of methane biosynthetic process from dimethyl sulfide [GO:1900342]; is a type of positive regulation of alkane biosynthetic process [GO:1901579]; is a type of positive regulation of cellular respiration [GO:1901857]; positively regulates methane biosynthetic process from dimethyl sulfide [GO:2001131] Definition: Any process that activates or increases the frequency, rate or extent of methane biosynthetic process from dimethyl sulfide. Sources: GOC:TermGenie, GOC:mengo_curators